short neuropeptide F receptor activity [GO:0036400] (molecular function) Relationships: is a type of neuropeptide receptor activity [GO:0008188] Also known as: sNPF receptor activity Definition: Combining with a short neuropeptide F and transmitting the signal within the cell to initiate a change in cell activity. Short neuropeptide F is an arthropod peptide of less than 28 residues (as small as 8-10 residues in some species) with a C-terminal RFamide or LRFamide. References: PMID:16330127, PMID:21440021 Sources: GOC:ha Note: Despite their naming, neuropeptide F (NPF) and short neuropeptide F (sNPF) are not closely related.